{
  "term_id": "UNKNOWN:0002",
  "term_label": "Unknown biological process",
  "gene": "UniProtKB:Q96C19",
  "gene_symbol": "EFHD2",
  "gene_name": "EF-hand domain-containing protein D2"
}